{
  "gene": "UniProtKB:P06734",
  "gene_name": "Low affinity immunoglobulin epsilon Fc receptor",
  "gene_symbol": "FCER2",
  "term_label": "carbohydrate binding",
  "term_id": "GO:0030246"
}